{
  "gene": "UniProtKB:Q96BK5",
  "gene_name": "PIN2_TERF1-interacting telomerase inhibitor 1",
  "term_id": "GO:0005730",
  "term_label": "nucleolus",
  "gene_symbol": "PINX1"
}